{
  "gene_name": "T-cell leukemia homeobox protein 3",
  "term_label": "nucleus",
  "gene_symbol": "TLX3",
  "term_id": "GO:0005634",
  "gene": "UniProtKB:O43711"
}